androsterone dehydrogenase [NAD(P)+] activity [GO:0047023] (molecular function) Sources: EC:1.1.1.209 Also known as: 3(17)alpha-hydroxysteroid dehydrogenase activity, 3(or 17)-alpha-hydroxysteroid dehydrogenase activity, 3(or 17)alpha-hydroxysteroid dehydrogenase activity, 3(or 17)alpha-hydroxysteroid:NAD(P)+ oxidoreductase activity Relationships: is a type of steroid dehydrogenase activity, acting on the CH-OH group of donors, NAD or NADP as acceptor [GO:0033764] Definition: Catalysis of the reaction: NAD(P)+ + androsterone = NAD(P)H + H+ + 5-alpha-androstane-3,17-dione.